{
  "gene_name": "Aryl hydrocarbon receptor",
  "gene_symbol": "AHR",
  "gene": "UniProtKB:P35869",
  "term_id": "GO:0006357",
  "term_label": "regulation of transcription by RNA polymerase II"
}